{
  "gene_symbol": "FOXA2",
  "gene_name": "Hepatocyte nuclear factor 3-beta",
  "term_label": "regulation of transcription by RNA polymerase II",
  "term_id": "GO:0006357",
  "gene": "UniProtKB:Q9Y261"
}